negative regulation of L-proline catabolic process to L-glutamate [GO:2001157] (biological process) Relationships: is a type of negative regulation of catabolic process [GO:0009895]; is a type of negative regulation of glutamate metabolic process [GO:2000212]; is a type of regulation of L-proline catabolic process to L-glutamate [GO:2001156]; negatively regulates L-proline catabolic process to L-glutamate [GO:0010133] Definition: Any process that stops, prevents or reduces the frequency, rate or extent of L-proline catabolic process to L-glutamate. Also known as: negative regulation of proline catabolic process to glutamate, negative regulation of proline breakdown to glutamate, negative regulation of proline degradation to glutamate, negative regulation of proline oxidation Sources: GOC:obol